{
  "gene": "UniProtKB:Q6VN20",
  "gene_symbol": "RANBP10",
  "term_id": "GO:0007010",
  "gene_name": "Ran-binding protein 10",
  "term_label": "cytoskeleton organization"
}